diterpenoid catabolic process [GO:0016103] (biological process) Definition: The chemical reactions and pathways resulting in the breakdown of diterpenoid compounds, terpenoids with four isoprene units. Sources: GOC:mah, ISBN:0198547684 Also known as: diterpenoid breakdown, diterpenoid catabolism, diterpenoid degradation, diterpene catabolic process, diterpene catabolism Relationships: is a type of GO:0016101; is a type of terpenoid catabolic process [GO:0016115] Subtypes: retinoic acid catabolic process [GO:0034653], gibberellin catabolic process [GO:0045487], 5alpha,9alpha,10beta-labda-8(20),13-dien-15-yl diphosphate catabolic process [GO:1901948], GO:1902242, GO:1902245